{
  "gene": "UniProtKB:A6NND4",
  "gene_symbol": "OR2AT4",
  "term_id": "GO:0007165",
  "gene_name": "Olfactory receptor 2AT4",
  "term_label": "signal transduction"
}